{
  "gene": "UniProtKB:Q8NDI1",
  "gene_symbol": "EHBP1",
  "term_label": "plasma membrane",
  "gene_name": "EH domain-binding protein 1",
  "term_id": "GO:0005886"
}